{
  "term_id": "GO:0003924",
  "gene_symbol": "GNAL",
  "gene_name": "Guanine nucleotide-binding protein G(olf) subunit alpha",
  "gene": "UniProtKB:P38405",
  "term_label": "GTPase activity"
}